NAD binding [GO:0051287] (molecular function) Definition: Binding to nicotinamide adenine dinucleotide, a coenzyme involved in many redox and biosynthetic reactions; binding may be to either the oxidized form, NAD+, or the reduced form, NADH. Sources: GOC:ai Also known as: nicotinamide adenine dinucleotide binding, NAD or NADH binding, NAD+ or NADH binding Relationships: is a type of adenyl nucleotide binding [GO:0030554] Subtypes: NAD+ binding [GO:0070403], NADH binding [GO:0070404]